{
  "gene_name": "Uncharacterized protein C8orf88",
  "term_label": "eukaryotic initiation factor 4E binding",
  "gene_symbol": "C8orf88",
  "gene": "UniProtKB:P0DMB2",
  "term_id": "GO:0008190"
}